{
  "gene": "UniProtKB:Q9HBH9",
  "term_id": "GO:0009931",
  "gene_name": "MAP kinase-interacting serine_threonine-protein kinase 2",
  "gene_symbol": "MKNK2",
  "term_label": "calcium-dependent protein serine/threonine kinase activity"
}